unfolded protein binding [GO:0051082] (molecular function) Relationships: is a type of GO:0005515 Also known as: chaperone activity Definition: Binding to an unfolded protein. Sources: GOC:ai